{
  "gene_symbol": "TAF1",
  "term_label": "RNA polymerase II general transcription initiation factor activity",
  "gene": "UniProtKB:P21675",
  "term_id": "GO:0016251",
  "gene_name": "Transcription initiation factor TFIID subunit 1"
}